{
  "gene": "UniProtKB:P01344",
  "term_label": "positive regulation of mitotic nuclear division",
  "term_id": "GO:0045840",
  "gene_name": "Insulin-like growth factor II",
  "gene_symbol": "IGF2"
}